{
  "gene_name": "Collagen alpha-2(V) chain",
  "gene": "UniProtKB:P05997",
  "term_label": "collagen fibril organization",
  "gene_symbol": "COL5A2",
  "term_id": "GO:0030199"
}